negative regulation of mitochondrial DNA replication [GO:0090298] (biological process) Relationships: is a type of regulation of mitochondrial DNA replication [GO:0090296]; is a type of negative regulation of mitochondrial DNA metabolic process [GO:1901859]; is a type of GO:2000104; negatively regulates mitochondrial DNA replication [GO:0006264] Sources: GOC:tb Definition: Any process that decreases the rate, frequency or extent of the process in which new strands of DNA are synthesized in the mitochondrion. Also known as: negative regulation of mitochondrial DNA synthesis